regulation of endocardial cushion to mesenchymal transition [GO:0140049] (biological process) Subtypes: negative regulation of endocardial cushion to mesenchymal transition [GO:0140050], positive regulation of endocardial cushion to mesenchymal transition [GO:0140051], regulation of endocardial cushion to mesenchymal transition involved in heart valve formation [GO:2000800] Definition: Any process that modulates the frequency, rate or extent of endocardial cushion to mesenchymal transition. References: PMID:21778427 Sources: GOC:BHF, GOC:BHF_miRNA, GOC:rph Relationships: is a type of regulation of cardiac epithelial to mesenchymal transition [GO:0062042]; regulates GO:0090500